{
  "term_label": "nucleus",
  "gene_symbol": "KRBOX4",
  "gene_name": "KRAB domain-containing protein 4",
  "term_id": "GO:0005634",
  "gene": "UniProtKB:Q5JUW0"
}